{
  "gene_symbol": "POTEB2",
  "gene": "UniProtKB:H3BUK9",
  "term_label": "Unknown molecular function",
  "term_id": "UNKNOWN:0001",
  "gene_name": "POTE ankyrin domain family member B2"
}